{
  "gene_symbol": "CD2",
  "term_label": "Unknown cellular component",
  "gene": "UniProtKB:P06729",
  "gene_name": "T-cell surface antigen CD2",
  "term_id": "UNKNOWN:0003"
}